perception of static position [GO:0019231] (biological process) Sources: ISBN:072168677X Relationships: is a type of proprioception [GO:0019230] Definition: The perception of the orientation of different parts of the body with respect to one another.